{
  "gene_name": "Nuclear receptor-interacting protein 1",
  "gene": "UniProtKB:P48552",
  "term_label": "transcription corepressor activity",
  "term_id": "GO:0003714",
  "gene_symbol": "NRIP1"
}